regulation of integrin biosynthetic process [GO:0045113] (biological process) Subtypes: regulation of beta 2 integrin biosynthetic process [GO:0045115], negative regulation of integrin biosynthetic process [GO:0045720], positive regulation of integrin biosynthetic process [GO:0045726] Also known as: regulation of integrin anabolism, regulation of integrin biosynthesis, regulation of integrin formation, regulation of integrin synthesis Sources: GOC:go_curators Relationships: is a type of GO:0010556; regulates integrin biosynthetic process [GO:0045112] Definition: Any process that modulates the frequency, rate or extent of the chemical reactions and pathways resulting in the formation of integrins.